farnesyl diphosphate kinase activity [GO:0047887] (molecular function) Relationships: is a type of kinase activity [GO:0016301]; is a type of phosphotransferase activity, phosphate group as acceptor [GO:0016776] Also known as: farnesyl-diphosphate kinase activity, ATP:farnesyl-diphosphate phosphotransferase activity, farnesyl pyrophosphate kinase activity Sources: RHEA:21544 Definition: Catalysis of the reaction: 2-trans,6-trans-farnesyl diphosphate + ATP = 2-trans,6-trans-farnesyl triphosphate + ADP.